{
  "gene_symbol": "CREB3L3",
  "term_id": "GO:0006357",
  "term_label": "regulation of transcription by RNA polymerase II",
  "gene": "UniProtKB:Q68CJ9",
  "gene_name": "Cyclic AMP-responsive element-binding protein 3-like protein 3"
}